{
  "gene": "UniProtKB:Q9ULW8",
  "term_label": "nucleus",
  "gene_name": "Protein-arginine deiminase type-3",
  "term_id": "GO:0005634",
  "gene_symbol": "PADI3"
}